{
  "term_id": "UNKNOWN:0002",
  "term_label": "Unknown biological process",
  "gene_symbol": "BTG4",
  "gene_name": "Protein BTG4",
  "gene": "UniProtKB:Q9NY30"
}